histone H4K8 deacetylase activity, hydrolytic mechanism [GO:0180033] (molecular function) References: PMID:37459529 Note: Note that the residue position corresponds to the canonical human H4 histone (UniProtKB:P02309); this residue is conserved across all eukaryotes. Note that the initiation methionine is cleaved, so the first residue is S1. Relationships: is a type of histone H4K deacetylase activity [GO:0141051]; is a type of histone deacetylase activity, hydrolytic mechanism [GO:0141221] Also known as: histone H4K48 deacetylase activity Definition: Catalysis of the reaction: histone H4 N6-acetyl-L-lysine (position 8) + H2O = histone H4 L-lysine (position 8) + acetate. This reaction represents the removal of an acetyl group from lysine at position 8 of the histone H4 protein.